regulation of postsynaptic density assembly [GO:0099151] (biological process) Relationships: is a type of regulation of postsynaptic specialization assembly [GO:0099150]; is a type of regulation of excitatory synapse assembly [GO:1904889]; is a type of regulation of postsynaptic density organization [GO:1905874]; regulates postsynaptic density assembly [GO:0097107] Definition: Any process that modulates the frequency, rate or extent of postsynaptic density assembly, the aggregation, arrangement and bonding together of a set of components to form a postsynaptic density. Sources: GOC:dos Subtypes: positive regulation of postsynaptic density assembly [GO:0160036], GO:0160037